mannose catabolic process [GO:0019309] (biological process) Relationships: is a type of GO:0006013; is a type of hexose catabolic process [GO:0019320] Sources: GOC:ai Definition: The chemical reactions and pathways resulting in the breakdown of mannose, the aldohexose manno-hexose, the C-2 epimer of glucose. Subtypes: GO:0061611, glycolytic process from mannose through fructose-6-phosphate [GO:0061619] Also known as: mannose breakdown, mannose catabolism, mannose degradation